vesicle transport along actin filament [GO:0030050] (biological process) Definition: Movement of a vesicle along an actin filament, mediated by motor proteins. Sources: GOC:mah Relationships: is a type of actin filament-based movement [GO:0030048]; is a type of actin filament-based transport [GO:0099515]; is a type of vesicle cytoskeletal trafficking [GO:0099518] Subtypes: synaptic vesicle transport along actin filament [GO:0099506]